{
  "gene": "UniProtKB:Q9HB14",
  "gene_name": "Potassium channel subfamily K member 13",
  "term_id": "GO:0022841",
  "gene_symbol": "KCNK13",
  "term_label": "potassium ion leak channel activity"
}